{
  "gene_name": "Olfactory receptor 6B3",
  "term_label": "olfactory receptor activity",
  "term_id": "GO:0004984",
  "gene": "UniProtKB:Q8NGW1",
  "gene_symbol": "OR6B3"
}